establishment of blood-nerve barrier [GO:0008065] (biological process) Relationships: is a type of endothelial cell development [GO:0001885]; is part of peripheral nervous system development [GO:0007422] Sources: GOC:dgh Also known as: establishment of blood/nerve barrier Definition: The establishment of the barrier between the perineurium of peripheral nerves and the vascular endothelium of endoneurial capillaries. The perineurium acts as a diffusion barrier, but ion permeability at the blood-nerve barrier is still higher than at the blood-brain barrier.